9-cis-retinoic acid metabolic process [GO:0042905] (biological process) Subtypes: 9-cis-retinoic acid biosynthetic process [GO:0042904] Definition: The chemical reactions and pathways involving 9-cis-retinoic acid, a metabolically active vitamin A derivative. Relationships: is a type of retinoic acid metabolic process [GO:0042573] References: PMID:11279029 Sources: GOC:jl Also known as: 9-cis-retinoic acid metabolism